{
  "gene": "UniProtKB:Q6ICL7",
  "gene_name": "Solute carrier family 35 member E4",
  "term_label": "antiporter activity",
  "term_id": "GO:0015297",
  "gene_symbol": "SLC35E4"
}